{
  "term_id": "UNKNOWN:0002",
  "term_label": "Unknown biological process",
  "gene_name": "Endogenous retrovirus group S71 member 1 Env polyprotein",
  "gene_symbol": "ERVS71-1",
  "gene": "UniProtKB:P61550"
}